transcription by RNA polymerase V [GO:0001060] (biological process) Regulation: regulated by regulation of transcription by RNA polymerase V [GO:1904279]; negatively regulated by negative regulation of transcription by RNA polymerase V [GO:1904280]; positively regulated by positive regulation of transcription by RNA polymerase V [GO:1904281] References: PMID:19110459 Sources: GOC:txnOH Definition: The synthesis of RNA from a DNA template by RNA polymerase V, originating at a Pol V-specific promoter. Also known as: transcription from RNA pol V promoter, transcription from RNA polymerase V promoter Relationships: is a type of DNA-templated transcription [GO:0006351]